cytokinin dehydrogenase activity [GO:0019139] (molecular function) Definition: Catalysis of the reaction: N6-dimethylallyladenine + acceptor + H2O = adenine + 3-methylbut-2-enal + reduced electron acceptor. Relationships: is a type of GO:0016645 Sources: EC:1.5.99.12 Note: Note that this term has a MetaCyc pathway reference as the pathway only has a single step. Also known as: 6-N-dimethylallyladenine:acceptor oxidoreductase activity, N6-dimethylallyladenine:(acceptor) oxidoreductase activity, N6-dimethylallyladenine:acceptor oxidoreductase activity, cytokinin oxidase activity